{
  "term_id": "GO:0004984",
  "gene_symbol": "OR52B4",
  "term_label": "olfactory receptor activity",
  "gene": "UniProtKB:Q8NGK2",
  "gene_name": "Olfactory receptor 52B4"
}